{
  "term_id": "GO:0009617",
  "term_label": "response to bacterium",
  "gene_name": "T cell receptor alpha chain constant",
  "gene": "UniProtKB:P01848",
  "gene_symbol": "TRAC"
}